transcription regulator complex [GO:0005667] (cellular component) Relationships: is a type of protein-containing complex [GO:0032991] Definition: A protein complex that is capable of associating with DNA by direct binding, or via other DNA-binding proteins or complexes, and regulating transcription. Subtypes: RNA polymerase I transcription regulator complex [GO:0000120], NuRD complex [GO:0016581], transcription repressor complex [GO:0017053], GO:0019185, Cbf1-Met4-Met28 complex [GO:0089713], RNA polymerase II transcription regulator complex [GO:0090575], RNA polymerase III transcription regulator complex [GO:0090576], GO:0090577, RNA polymerase V transcription regulator complex [GO:0090578], sigma factor antagonist complex [GO:1903865], ModE complex [GO:1990198], CHOP-ATF3 complex [GO:1990622] Also known as: cytoplasmic transcription factor complex, nuclear transcription factor complex, transcription factor complex Sources: GOC:jl